cell envelope organization [GO:0043163] (biological process) Also known as: cell envelope organisation, cell envelope organization and biogenesis Sources: GOC:jl Definition: A process that is carried out at the cellular level which results in the assembly, arrangement of constituent parts, or disassembly of the cell envelope, everything external to, but not including, the cytoplasmic membrane of bacteria, encompassing the periplasmic space, cell wall, and outer membrane if present. Relationships: is a type of external encapsulating structure organization [GO:0045229]